{
  "gene": "UniProtKB:Q9NQ60",
  "gene_symbol": "EQTN",
  "term_id": "GO:0002079",
  "gene_name": "Equatorin",
  "term_label": "inner acrosomal membrane"
}